{
  "gene_symbol": "NHEJ1",
  "term_id": "GO:0032807",
  "term_label": "DNA ligase IV complex",
  "gene": "UniProtKB:Q9H9Q4",
  "gene_name": "Non-homologous end-joining factor 1"
}